{
  "term_label": "calcium channel activity",
  "term_id": "GO:0005262",
  "gene_name": "Sodium_potassium_calcium exchanger 1",
  "gene_symbol": "SLC24A1",
  "gene": "UniProtKB:O60721"
}